{
  "gene_name": "WAS protein family homolog 2",
  "term_label": "Arp2/3 complex-mediated actin nucleation",
  "gene": "UniProtKB:Q6VEQ5",
  "term_id": "GO:0034314",
  "gene_symbol": "WASH2P"
}